{
  "term_id": "GO:0005886",
  "gene_name": "Olfactory receptor 4Q2",
  "term_label": "plasma membrane",
  "gene": "UniProtKB:P0C623",
  "gene_symbol": "OR4Q2"
}